{
  "gene": "UniProtKB:Q5JWF2",
  "term_id": "GO:0035255",
  "gene_name": "Guanine nucleotide-binding protein G(s) subunit alpha isoforms XLas",
  "gene_symbol": "GNAS",
  "term_label": "ionotropic glutamate receptor binding"
}